{
  "term_label": "cytosol",
  "term_id": "GO:0005829",
  "gene_name": "Histone deacetylase 6",
  "gene": "UniProtKB:Q9UBN7",
  "gene_symbol": "HDAC6"
}